{
  "term_label": "Unknown cellular component",
  "gene_name": "Ribonuclease pancreatic",
  "gene_symbol": "RNASE1",
  "term_id": "UNKNOWN:0003",
  "gene": "UniProtKB:P07998"
}